postsynaptic membrane organization [GO:0001941] (biological process) Definition: A process which results in the assembly, arrangement of constituent parts, or disassembly of a postsynaptic membrane, the specialized area of membrane facing the presynaptic membrane on the tip of the nerve ending and separated from it by a minute cleft (the synaptic cleft). Sources: GOC:dph, GOC:pr Also known as: post-synaptic membrane organization, postsynaptic membrane organisation Relationships: is a type of GO:0061024; is part of GO:0099173 Subtypes: GO:0097104 Regulation: regulated by GO:1901626; RO_0002212 by negative regulation of postsynaptic membrane organization [GO:1901627]; positively regulated by positive regulation of postsynaptic membrane organization [GO:1901628]